{
  "gene_name": "Zinc finger protein 446",
  "term_label": "Unknown cellular component",
  "gene_symbol": "ZNF446",
  "term_id": "UNKNOWN:0003",
  "gene": "UniProtKB:Q9NWS9"
}